{
  "term_id": "GO:0005634",
  "gene_symbol": "API5",
  "gene": "UniProtKB:Q9BZZ5",
  "gene_name": "Apoptosis inhibitor 5",
  "term_label": "nucleus"
}